{
  "gene_name": "Putative serine_threonine-protein phosphatase 4 regulatory subunit 1-like",
  "term_label": "Unknown molecular function",
  "gene": "UniProtKB:Q9P1A2",
  "term_id": "UNKNOWN:0001",
  "gene_symbol": "PPP4R1L"
}